{
  "term_id": "GO:0032024",
  "gene_name": "Neuronatin",
  "gene_symbol": "NNAT",
  "term_label": "positive regulation of insulin secretion",
  "gene": "UniProtKB:Q16517"
}